{
  "gene": "UniProtKB:Q96T51",
  "term_id": "GO:0005737",
  "gene_symbol": "RUFY1",
  "term_label": "cytoplasm",
  "gene_name": "RUN and FYVE domain-containing protein 1"
}